negative regulation of nuclear division [GO:0051784] (biological process) Subtypes: GO:0045835, GO:0045839 Sources: GOC:ai Definition: Any process that stops, prevents, or reduces the frequency, rate or extent of nuclear division, the partitioning of the nucleus and its genetic information. Also known as: down regulation of nuclear division, down-regulation of nuclear division, downregulation of nuclear division, inhibition of nuclear division Relationships: is a type of negative regulation of organelle organization [GO:0010639]; is a type of GO:0051783; negatively regulates nuclear division [GO:0000280]